xanthine catabolic process [GO:0009115] (biological process) Definition: The chemical reactions and pathways resulting in the breakdown of xanthine, 2,6-dihydroxypurine, a purine formed in the metabolic breakdown of guanine but not present in nucleic acids. Sources: GOC:go_curators Also known as: xanthine breakdown, xanthine catabolism, xanthine degradation, xanthine oxidation Relationships: is a type of GO:0006145; is a type of xanthine metabolic process [GO:0046110]